platelet dense granule [GO:0042827] (cellular component) Relationships: is a type of secretory granule [GO:0030141] Definition: Electron-dense granule occurring in blood platelets that stores and secretes adenosine nucleotides and serotonin. They contain a highly condensed core consisting of serotonin, histamine, calcium, magnesium, ATP, ADP, pyrophosphate and membrane lysosomal proteins. Also known as: bull's eye body, platelet dense body References: PMID:10403682, PMID:11487378 Sources: GOC:jl